{
  "term_label": "CCR4-NOT complex binding",
  "gene": "UniProtKB:Q9Y4F3",
  "gene_name": "Meiosis regulator and mRNA stability factor 1",
  "term_id": "GO:1905762",
  "gene_symbol": "MARF1"
}